{
  "gene_symbol": "COQ10B",
  "term_id": "UNKNOWN:0002",
  "gene": "UniProtKB:Q9H8M1",
  "term_label": "Unknown biological process",
  "gene_name": "Coenzyme Q-binding protein COQ10 homolog B, mitochondrial"
}